{
  "term_id": "GO:0045109",
  "gene": "UniProtKB:O43790",
  "term_label": "intermediate filament organization",
  "gene_name": "Keratin, type II cuticular Hb6",
  "gene_symbol": "KRT86"
}